{
  "term_id": "GO:0005737",
  "gene_symbol": "PADI1",
  "gene_name": "Protein-arginine deiminase type-1",
  "term_label": "cytoplasm",
  "gene": "UniProtKB:Q9ULC6"
}